{
  "gene_name": "Small ribosomal subunit protein uS2",
  "term_id": "GO:0003735",
  "gene_symbol": "RPSA",
  "term_label": "structural constituent of ribosome",
  "gene": "UniProtKB:P08865"
}